{
  "term_id": "GO:0060259",
  "gene_name": "Orexigenic neuropeptide QRFP",
  "gene": "UniProtKB:P83859",
  "gene_symbol": "QRFP",
  "term_label": "regulation of feeding behavior"
}